{
  "gene_name": "Probable E3 ubiquitin-protein ligase HECTD4",
  "gene_symbol": "HECTD4",
  "term_id": "UNKNOWN:0003",
  "term_label": "Unknown cellular component",
  "gene": "UniProtKB:Q9Y4D8"
}